{
  "gene": "UniProtKB:Q969V6",
  "gene_symbol": "MRTFA",
  "term_id": "GO:0003713",
  "gene_name": "Myocardin-related transcription factor A",
  "term_label": "transcription coactivator activity"
}